{
  "gene": "UniProtKB:Q13349",
  "gene_symbol": "ITGAD",
  "term_id": "GO:0008305",
  "term_label": "integrin complex",
  "gene_name": "Integrin alpha-D"
}